{
  "term_id": "UNKNOWN:0001",
  "gene_name": "Immunoglobulin kappa variable 3-11",
  "gene": "UniProtKB:P04433",
  "gene_symbol": "IGKV3-11",
  "term_label": "Unknown molecular function"
}